{
  "gene_name": "Aflatoxin B1 aldehyde reductase member 4",
  "term_label": "cytoplasm",
  "term_id": "GO:0005737",
  "gene_symbol": "AKR7L",
  "gene": "UniProtKB:Q8NHP1"
}